{
  "term_id": "GO:0022625",
  "gene_name": "Large ribosomal subunit protein eL6",
  "term_label": "cytosolic large ribosomal subunit",
  "gene_symbol": "RPL6",
  "gene": "UniProtKB:Q02878"
}